{
  "term_label": "extracellular space",
  "gene": "UniProtKB:Q8IWY4",
  "term_id": "GO:0005615",
  "gene_symbol": "SCUBE1",
  "gene_name": "Signal peptide, CUB and EGF-like domain-containing protein 1"
}